specification of stamen identity [GO:0010097] (biological process) Definition: The process in which a floral organ primordium acquires stamen or staminode identity. Identity is considered to be the aggregate of characteristics by which a structure is recognized. Sources: GOC:tair_curators Relationships: is a type of specification of floral organ identity [GO:0010093]; is part of stamen formation [GO:0048455]